{
  "term_id": "GO:0005829",
  "gene_name": "UBX domain-containing protein 2A",
  "gene": "UniProtKB:P68543",
  "term_label": "cytosol",
  "gene_symbol": "UBXN2A"
}